{
  "gene_symbol": "LHPP",
  "term_label": "phosphatase activity",
  "term_id": "GO:0016791",
  "gene": "UniProtKB:Q9H008",
  "gene_name": "Phospholysine phosphohistidine inorganic pyrophosphate phosphatase"
}